{
  "gene_name": "High affinity immunoglobulin epsilon receptor subunit alpha",
  "term_id": "GO:0009897",
  "gene": "UniProtKB:P12319",
  "term_label": "external side of plasma membrane",
  "gene_symbol": "FCER1A"
}